{
  "gene_name": "Prostacyclin receptor",
  "gene": "UniProtKB:P43119",
  "gene_symbol": "PTGIR",
  "term_id": "GO:0007189",
  "term_label": "adenylate cyclase-activating G protein-coupled receptor signaling pathway"
}